{
  "gene": "UniProtKB:Q494R4",
  "gene_name": "Coiled-coil domain-containing protein 153",
  "gene_symbol": "CCDC153",
  "term_id": "UNKNOWN:0003",
  "term_label": "Unknown cellular component"
}